C-X3-C chemokine binding [GO:0019960] (molecular function) Relationships: is a type of GO:0019956 Sources: GOC:ai Definition: Binding to a C-X3-C chemokine; C-X3-C chemokines have three amino acids between the first two cysteines of the characteristic four-cysteine motif.